MHC class Ib protein binding [GO:0023029] (MF) Relationships: is a type of MHC protein binding [GO:0042287] Subtypes: MHC class Ib protein binding, via antigen binding groove [GO:0023030], MHC class Ib protein binding, via lateral surface [GO:0023031] Sources: GOC:mtg_signal, GOC:vw Definition: Binding to a major histocompatibility complex class Ib molecules.